{
  "term_label": "negative regulation of neuron differentiation",
  "gene": "UniProtKB:Q13127",
  "term_id": "GO:0045665",
  "gene_symbol": "REST",
  "gene_name": "RE1-silencing transcription factor"
}